{
  "term_id": "GO:0000724",
  "gene": "UniProtKB:O60921",
  "gene_name": "Checkpoint protein HUS1",
  "gene_symbol": "HUS1",
  "term_label": "double-strand break repair via homologous recombination"
}